pancreatic trypsinogen secretion [GO:1990747] (biological process) Definition: The regulated release of trypsinogen from the cells of the exocrine pancreas. References: PMID:12771515 Also known as: pancreatic trypsinogen release Relationships: is_a protein secretion [GO:0009306]; is part of GO:0030157 Regulation: regulated by GO:1904242; negatively regulated by negative regulation of pancreatic trypsinogen secretion [GO:1904243]; positively regulated by positive regulation of pancreatic trypsinogen secretion [GO:1904244]